T cell anergy [GO:0002870] (biological process) Definition: Any process contributing to anergy in T cells, a state of functional inactivation which is part of T cell tolerance induction. Sources: GOC:add, ISBN:0781735149 Also known as: T lymphocyte anergy, T-cell anergy, T-lymphocyte anergy Relationships: is a type of lymphocyte anergy [GO:0002249]; is a type of GO:0002517 Regulation: regulated by regulation of T cell anergy [GO:0002667]; negatively regulated by negative regulation of T cell anergy [GO:0002668]; positively regulated by positive regulation of T cell anergy [GO:0002669]